{
  "gene": "UniProtKB:Q16787",
  "term_label": "signal transduction",
  "gene_symbol": "LAMA3",
  "gene_name": "Laminin subunit alpha-3",
  "term_id": "GO:0007165"
}